regulation of eating behavior [GO:1903998] (biological process) Subtypes: regulation of nematode pharyngeal pumping [GO:0043051], negative regulation of eating behavior [GO:1903999], positive regulation of eating behavior [GO:1904000] Definition: Any process that modulates the frequency, rate or extent of eating behavior. Relationships: is a type of regulation of feeding behavior [GO:0060259]; RO_0002211 eating behavior [GO:0042755] References: PMID:11961051 Sources: GOC:TermGenie, GO_REF:0000058 Also known as: regulation of eating behaviour